{
  "term_label": "plasma membrane",
  "term_id": "GO:0005886",
  "gene_symbol": "TLR1",
  "gene_name": "Toll-like receptor 1",
  "gene": "UniProtKB:Q15399"
}